{
  "gene_name": "Centriolar coiled-coil protein of 110 kDa",
  "term_id": "UNKNOWN:0001",
  "gene_symbol": "CCP110",
  "gene": "UniProtKB:O43303",
  "term_label": "Unknown molecular function"
}